{
  "gene_symbol": "OR56B4",
  "gene_name": "Olfactory receptor 56B4",
  "term_label": "olfactory receptor activity",
  "term_id": "GO:0004984",
  "gene": "UniProtKB:Q8NH76"
}